{
  "term_id": "GO:0005737",
  "gene": "UniProtKB:Q8WUY3",
  "term_label": "cytoplasm",
  "gene_name": "Protein prune homolog 2",
  "gene_symbol": "PRUNE2"
}